{
  "gene": "UniProtKB:Q92624",
  "term_id": "GO:1990756",
  "gene_symbol": "APPBP2",
  "gene_name": "Amyloid protein-binding protein 2",
  "term_label": "ubiquitin-like ligase-substrate adaptor activity"
}